regulation of stem cell differentiation [GO:2000736] (biological process) Definition: Any process that modulates the frequency, rate or extent of stem cell differentiation. Sources: GOC:obol Relationships: is a type of regulation of cell differentiation [GO:0045595]; regulates stem cell differentiation [GO:0048863] Subtypes: regulation of cardioblast differentiation [GO:0051890], regulation of hematopoietic stem cell differentiation [GO:1902036], regulation of neural crest cell differentiation [GO:1905292], negative regulation of stem cell differentiation [GO:2000737], GO:2000738, regulation of mesenchymal stem cell differentiation [GO:2000739]